{
  "gene_symbol": "OR56B1",
  "term_id": "UNKNOWN:0002",
  "gene": "UniProtKB:Q8NGI3",
  "term_label": "Unknown biological process",
  "gene_name": "Olfactory receptor 56B1"
}